{
  "term_label": "anaphase-promoting complex",
  "gene_name": "Cell division cycle protein 23 homolog",
  "gene": "UniProtKB:Q9UJX2",
  "gene_symbol": "CDC23",
  "term_id": "GO:0005680"
}